{
  "term_label": "myosin II binding",
  "term_id": "GO:0045159",
  "gene": "UniProtKB:Q5T5C0",
  "gene_symbol": "STXBP5",
  "gene_name": "Syntaxin-binding protein 5"
}